{
  "gene_name": "Glutamate dehydrogenase 1, mitochondrial",
  "term_id": "GO:0005739",
  "term_label": "mitochondrion",
  "gene_symbol": "GLUD1",
  "gene": "UniProtKB:P00367"
}